{
  "term_id": "GO:0007157",
  "term_label": "heterophilic cell-cell adhesion",
  "gene_symbol": "CRB1",
  "gene": "UniProtKB:P82279",
  "gene_name": "Protein crumbs homolog 1"
}